{
  "term_id": "GO:0005634",
  "gene_symbol": "NR6A1",
  "gene": "UniProtKB:Q15406",
  "term_label": "nucleus",
  "gene_name": "Nuclear receptor subfamily 6 group A member 1"
}